{
  "term_id": "GO:0005179",
  "gene": "UniProtKB:P48304",
  "term_label": "hormone activity",
  "gene_name": "Lithostathine-1-beta",
  "gene_symbol": "REG1B"
}